{
  "gene_symbol": "NRARP",
  "gene_name": "Notch-regulated ankyrin repeat-containing protein",
  "gene": "UniProtKB:Q7Z6K4",
  "term_label": "blood vessel endothelial cell proliferation involved in sprouting angiogenesis",
  "term_id": "GO:0002043"
}